{
  "gene_symbol": "PCDHGB6",
  "gene": "UniProtKB:Q9Y5F9",
  "term_id": "GO:0005886",
  "gene_name": "Protocadherin gamma-B6",
  "term_label": "plasma membrane"
}